{
  "gene_name": "Tubulin beta-1 chain",
  "term_label": "microtubule",
  "term_id": "GO:0005874",
  "gene_symbol": "TUBB1",
  "gene": "UniProtKB:Q9H4B7"
}